{
  "gene": "UniProtKB:Q52M93",
  "term_id": "GO:0006357",
  "term_label": "regulation of transcription by RNA polymerase II",
  "gene_name": "Zinc finger protein 585B",
  "gene_symbol": "ZNF585B"
}